{
  "term_id": "GO:0005886",
  "gene": "UniProtKB:O43306",
  "gene_symbol": "ADCY6",
  "term_label": "plasma membrane",
  "gene_name": "Adenylate cyclase type 6"
}